L-DOPA binding [GO:0072544] (molecular function) Definition: Binding to L-DOPA, the modified amino acid (2S)-2-amino-3-(3,4-dihydroxyphenyl)propanoic acid. Relationships: is a type of amino acid binding [GO:0016597]; is a type of carboxylic acid binding [GO:0031406]; is a type of GO:0072341 Sources: GOC:mah, GOC:vw